{
  "term_label": "RNA polymerase II cis-regulatory region sequence-specific DNA binding",
  "gene": "UniProtKB:Q86XU0",
  "gene_name": "Zinc finger protein 677",
  "term_id": "GO:0000978",
  "gene_symbol": "ZNF677"
}